aliphatic amine dehydrogenase activity [GO:0030058] (molecular function) Subtypes: aliphatic amine oxidase activity [GO:0052595] Also known as: amine dehydrogenase activity, primary-amine dehydrogenase activity, MADH activity, amine: (acceptor) oxidoreductase (deaminating), methylamine dehydrogenase activity, primary-amine:acceptor oxidoreductase (deaminating) Sources: RHEA:51128 Relationships: is a type of oxidoreductase activity, acting on the CH-NH2 group of donors [GO:0016638] Definition: Catalysis of the reaction: an aliphatic amine + an acceptor (A) + H2O = an aldehyde + a reduced acceptor (AH2) + NH4+.